chiasma assembly [GO:0051026] (biological process) Relationships: is a type of cellular component assembly [GO:0022607]; is a type of meiotic cell cycle process [GO:1903046]; is part of homologous chromosome pairing at meiosis [GO:0007129]; is part of GO:0007131 Definition: The cell cycle process in which a connection between chromatids assembles, indicating where an exchange of homologous segments has taken place by the crossing-over of non-sister chromatids. References: PMID:23396135